{
  "gene_symbol": "PRSS55",
  "gene_name": "Serine protease 55",
  "term_id": "GO:0016485",
  "term_label": "protein processing",
  "gene": "UniProtKB:Q6UWB4"
}